{
  "gene_name": "Cysteine-rich protein 3",
  "term_label": "Unknown cellular component",
  "gene_symbol": "CRIP3",
  "gene": "UniProtKB:Q6Q6R5",
  "term_id": "UNKNOWN:0003"
}